L-glutamate transmembrane import into vacuole [GO:0090515] (biological process) Definition: The directed movement of L-glutamate into the vacuole across the vacuolar membrane. Sources: GOC:al Relationships: is a type of GO:0015813; is a type of GO:0090454